{
  "gene_name": "Conserved oligomeric Golgi complex subunit 3",
  "term_id": "GO:0017119",
  "gene_symbol": "COG3",
  "gene": "UniProtKB:Q96JB2",
  "term_label": "Golgi transport complex"
}